{
  "gene_symbol": "TADA2A",
  "gene_name": "Transcriptional adapter 2-alpha",
  "term_label": "regulation of transcription by RNA polymerase II",
  "gene": "UniProtKB:O75478",
  "term_id": "GO:0006357"
}